{
  "term_id": "GO:1904491",
  "gene_name": "Tectonic-1",
  "term_label": "protein localization to ciliary transition zone",
  "gene_symbol": "TCTN1",
  "gene": "UniProtKB:Q2MV58"
}